{
  "gene": "UniProtKB:Q9UKJ3",
  "term_label": "nucleus",
  "gene_name": "G patch domain-containing protein 8",
  "term_id": "GO:0005634",
  "gene_symbol": "GPATCH8"
}